{
  "gene_symbol": "ZIC5",
  "gene_name": "Zinc finger protein ZIC 5",
  "term_id": "GO:0000981",
  "term_label": "DNA-binding transcription factor activity, RNA polymerase II-specific",
  "gene": "UniProtKB:Q96T25"
}